pre-mRNA intronic binding [GO:0097157] (molecular function) Subtypes: pre-mRNA intronic pyrimidine-rich binding [GO:0097158] Relationships: is a type of pre-mRNA binding [GO:0036002] Also known as: pre-mRNA intron binding, pre-messenger RNA intronic binding References: PMID:16260624 Sources: GOC:ans Definition: Binding to an intronic sequence of a pre-messenger RNA (pre-mRNA).